{
  "gene_symbol": "RIPPLY1",
  "gene_name": "Protein ripply1",
  "gene": "UniProtKB:Q0D2K3",
  "term_id": "GO:0009880",
  "term_label": "embryonic pattern specification"
}